{
  "gene": "UniProtKB:P40763",
  "term_label": "cell surface receptor signaling pathway via JAK-STAT",
  "term_id": "GO:0007259",
  "gene_name": "Signal transducer and activator of transcription 3",
  "gene_symbol": "STAT3"
}